termination of T cell signal transduction [GO:0023022] (biological process) Definition: The signaling process in which T cell signal transduction is brought to an end rather than being reversibly modulated. Sources: GOC:mtg_signal Relationships: is a type of termination of signal transduction [GO:0023021]; is a type of negative regulation of T cell receptor signaling pathway [GO:0050860]; is part of T cell receptor signaling pathway [GO:0050852]